{
  "gene_name": "SLIT and NTRK-like protein 6",
  "gene_symbol": "SLITRK6",
  "gene": "UniProtKB:Q9H5Y7",
  "term_label": "Unknown molecular function",
  "term_id": "UNKNOWN:0001"
}